{
  "term_id": "GO:0036503",
  "term_label": "ERAD pathway",
  "gene_name": "F-box only protein 6",
  "gene": "UniProtKB:Q9NRD1",
  "gene_symbol": "FBXO6"
}